{
  "gene": "UniProtKB:A0A075B6J1",
  "term_label": "immunoglobulin complex",
  "gene_symbol": "IGLV5-37",
  "gene_name": "Immunoglobulin lambda variable 5-37",
  "term_id": "GO:0019814"
}